{
  "term_label": "Unknown biological process",
  "gene_name": "Putative uncharacterized protein FLJ44672",
  "gene_symbol": "Q6ZQT7",
  "gene": "UniProtKB:Q6ZQT7",
  "term_id": "UNKNOWN:0002"
}